{
  "gene_symbol": "DNAAF4",
  "gene_name": "Dynein axonemal assembly factor 4",
  "gene": "UniProtKB:Q8WXU2",
  "term_id": "GO:0036159",
  "term_label": "inner dynein arm assembly"
}